{
  "gene_name": "Small lysine-rich protein 1",
  "term_id": "UNKNOWN:0003",
  "term_label": "Unknown cellular component",
  "gene": "UniProtKB:H3BMG3",
  "gene_symbol": "SMKR1"
}